{
  "gene_name": "Phorbol-12-myristate-13-acetate-induced protein 1",
  "term_label": "Unknown biological process",
  "gene_symbol": "PMAIP1",
  "gene": "UniProtKB:Q13794",
  "term_id": "UNKNOWN:0002"
}